negative regulation of vascular endothelial growth factor receptor signaling pathway [GO:0030948] (biological process) Definition: Any process that stops, prevents, or reduces the frequency, rate or extent of vascular endothelial growth factor receptor signaling pathway activity. Relationships: is a type of negative regulation of signal transduction [GO:0009968]; is a type of regulation of vascular endothelial growth factor receptor signaling pathway [GO:0030947]; is a type of negative regulation of cellular response to growth factor stimulus [GO:0090288]; negatively regulates vascular endothelial growth factor receptor signaling pathway [GO:0048010] Sources: GOC:dgh Also known as: down regulation of vascular endothelial growth factor receptor signaling pathway, down-regulation of vascular endothelial growth factor receptor signaling pathway, downregulation of vascular endothelial growth factor receptor signaling pathway, negative regulation of VEGF receptor signaling pathway, negative regulation of VEGF receptor signalling pathway, negative regulation of vascular endothelial growth factor receptor signalling pathway, inhibition of vascular endothelial growth factor receptor signaling pathway